{
  "gene_name": "Glycogen phosphorylase, liver form",
  "term_label": "pyridoxal phosphate binding",
  "gene_symbol": "PYGL",
  "gene": "UniProtKB:P06737",
  "term_id": "GO:0030170"
}